positive regulation of phospholipase C/protein kinase C signal transduction [GO:0141214] (biological process) Also known as: positive regulation of PLC/PKC signal transduction Relationships: is a type of positive regulation of intracellular signal transduction [GO:1902533]; positively regulates phospholipase C/protein kinase C signal transduction [GO:0141212] Definition: Any process that activates or increases the frequency, rate or extent of phospholipase C/protein kinase C signal transduction. References: PMID:24008408, PMID:32255775